{
  "term_label": "plasma membrane",
  "gene": "UniProtKB:P43657",
  "term_id": "GO:0005886",
  "gene_name": "Lysophosphatidic acid receptor 6",
  "gene_symbol": "LPAR6"
}